{
  "term_id": "GO:0005829",
  "gene_name": "NADPH--cytochrome P450 reductase",
  "gene_symbol": "POR",
  "gene": "UniProtKB:P16435",
  "term_label": "cytosol"
}